regulation of single-species biofilm formation [GO:1900190] (biological process) Relationships: is a type of regulation of cellular process [GO:0050794]; regulates single-species biofilm formation [GO:0044010] Sources: GOC:TermGenie, GOC:di Subtypes: negative regulation of single-species biofilm formation [GO:1900191], positive regulation of single-species biofilm formation [GO:1900192], regulation of single-species biofilm formation in or on host organism [GO:1900228], GO:1900231 Definition: Any process that modulates the frequency, rate or extent of single-species biofilm formation.